{
  "term_id": "GO:0099175",
  "gene": "UniProtKB:Q6PCB6",
  "gene_name": "Alpha_beta hydrolase domain-containing protein 17C",
  "term_label": "regulation of postsynapse organization",
  "gene_symbol": "ABHD17C"
}